{
  "gene_name": "Serine protease HTRA2, mitochondrial",
  "gene": "UniProtKB:O43464",
  "term_label": "serine-type endopeptidase activity",
  "term_id": "GO:0004252",
  "gene_symbol": "HTRA2"
}